{
  "term_label": "extracellular space",
  "gene_symbol": "CLEC11A",
  "gene_name": "C-type lectin domain family 11 member A",
  "term_id": "GO:0005615",
  "gene": "UniProtKB:Q9Y240"
}